{
  "gene_symbol": "SPHK2",
  "gene": "UniProtKB:Q9NRA0",
  "gene_name": "Sphingosine kinase 2",
  "term_id": "GO:0043065",
  "term_label": "positive regulation of apoptotic process"
}